{
  "gene_symbol": "ANKZF1",
  "gene_name": "tRNA endonuclease ANKZF1",
  "term_label": "ERAD pathway",
  "term_id": "GO:0036503",
  "gene": "UniProtKB:Q9H8Y5"
}